endochitinase activity [GO:0008843] (molecular function) Relationships: is a type of chitinase activity [GO:0004568] References: PMID:11468293 Sources: EC:3.2.1.14, GOC:bf, GOC:kah, GOC:pde Also known as: 1,4-beta-poly-N-acetylglucosaminidase, chitinase, chitodextrinase, poly-beta-glucosaminidase Definition: Catalysis of the hydrolysis of nonterminal (1->4)-beta linkages of N-acetyl-D-glucosamine (GlcNAc) polymers of chitin and chitodextrins. Typically, endochitinases cleave randomly within the chitin chain.